{
  "term_id": "GO:0030139",
  "term_label": "endocytic vesicle",
  "gene_symbol": "EHD3",
  "gene": "UniProtKB:Q9NZN3",
  "gene_name": "EH domain-containing protein 3"
}